{
  "gene_name": "NEDD8",
  "gene": "UniProtKB:Q15843",
  "term_label": "modification-dependent protein catabolic process",
  "gene_symbol": "NEDD8",
  "term_id": "GO:0019941"
}